{
  "term_label": "nucleus",
  "gene_name": "Probable ATP-dependent RNA helicase DDX5",
  "gene_symbol": "DDX5",
  "term_id": "GO:0005634",
  "gene": "UniProtKB:P17844"
}